{
  "term_label": "non-motile cilium assembly",
  "gene_name": "X-linked retinitis pigmentosa GTPase regulator-interacting protein 1",
  "term_id": "GO:1905515",
  "gene": "UniProtKB:Q96KN7",
  "gene_symbol": "RPGRIP1"
}